{
  "gene_name": "Sarcospan",
  "gene": "UniProtKB:Q14714",
  "gene_symbol": "SSPN",
  "term_id": "GO:0042383",
  "term_label": "sarcolemma"
}